{
  "gene": "UniProtKB:P26045",
  "gene_name": "Tyrosine-protein phosphatase non-receptor type 3",
  "gene_symbol": "PTPN3",
  "term_label": "protein tyrosine phosphatase activity",
  "term_id": "GO:0004725"
}